{
  "gene": "UniProtKB:Q02297",
  "term_label": "peripheral nervous system development",
  "term_id": "GO:0007422",
  "gene_symbol": "NRG1",
  "gene_name": "Pro-neuregulin-1, membrane-bound isoform"
}